{
  "gene_symbol": "ADORA1",
  "term_id": "GO:0007186",
  "gene": "UniProtKB:P30542",
  "gene_name": "Adenosine receptor A1",
  "term_label": "G protein-coupled receptor signaling pathway"
}